{
  "term_label": "U2-type spliceosomal complex",
  "gene_name": "HIV Tat-specific factor 1",
  "term_id": "GO:0005684",
  "gene_symbol": "HTATSF1",
  "gene": "UniProtKB:O43719"
}